{
  "term_id": "UNKNOWN:0001",
  "gene_name": "Zinc finger MYND domain-containing protein 10",
  "term_label": "Unknown molecular function",
  "gene": "UniProtKB:O75800",
  "gene_symbol": "ZMYND10"
}